{
  "term_label": "Unknown molecular function",
  "gene_name": "Putative lipocalin 1-like protein 1",
  "gene": "UniProtKB:Q5VSP4",
  "term_id": "UNKNOWN:0001",
  "gene_symbol": "LCN1P1"
}